{
  "term_id": "GO:0009986",
  "term_label": "cell surface",
  "gene": "UniProtKB:O95944",
  "gene_name": "Natural cytotoxicity triggering receptor 2",
  "gene_symbol": "NCR2"
}